stereocilia coupling link [GO:0002139] (cellular component) Subtypes: stereocilia tip link [GO:0002140], stereocilia ankle link [GO:0002141] Definition: A structure involved in coupling stereocilia to one another in sensory hair cells There are four morphologically distinct types: tip links, horizontal top connectors, shaft connectors and ankle links. Tip links and horizontal top connectors are the only inter-stereocilia links associated with mature cochlea, whereas ankle links appear during development of the auditory hair bundle. References: PMID:16775142 Relationships: is a type of cellular anatomical structure [GO:0110165]; is part of stereocilium bundle [GO:0032421]